{
  "term_id": "GO:0005634",
  "gene_symbol": "ADAT3",
  "term_label": "nucleus",
  "gene": "UniProtKB:Q96EY9",
  "gene_name": "Probable inactive tRNA-specific adenosine deaminase-like protein 3"
}